{
  "gene_symbol": "IMPDH2",
  "gene": "UniProtKB:P12268",
  "gene_name": "Inosine-5'-monophosphate dehydrogenase 2",
  "term_id": "GO:0003938",
  "term_label": "IMP dehydrogenase activity"
}